regulation of fatty acid oxidation [GO:0046320] (biological process) Relationships: is a type of GO:0019217; regulates GO:0019395 Subtypes: regulation of fatty acid beta-oxidation [GO:0031998], GO:0046321, GO:0046322 Sources: GOC:ai Definition: Any process that modulates the frequency, rate or extent of fatty acid oxidation.